{
  "gene": "UniProtKB:Q8TER5",
  "term_id": "GO:0005085",
  "term_label": "guanyl-nucleotide exchange factor activity",
  "gene_symbol": "ARHGEF40",
  "gene_name": "Rho guanine nucleotide exchange factor 40"
}